{
  "term_id": "GO:0032153",
  "term_label": "cell division site",
  "gene": "UniProtKB:Q92599",
  "gene_name": "Septin-8",
  "gene_symbol": "SEPTIN8"
}